{
  "gene_name": "Receptor-interacting serine_threonine-protein kinase 3",
  "term_label": "cytoplasm",
  "term_id": "GO:0005737",
  "gene": "UniProtKB:Q9Y572",
  "gene_symbol": "RIPK3"
}